{
  "term_label": "intracellular potassium ion homeostasis",
  "gene_name": "Sodium_potassium-transporting ATPase subunit alpha-1",
  "gene_symbol": "ATP1A1",
  "term_id": "GO:0030007",
  "gene": "UniProtKB:P05023"
}